{
  "gene_symbol": "TRIM16",
  "gene_name": "Tripartite motif-containing protein 16",
  "term_label": "Unknown biological process",
  "term_id": "UNKNOWN:0002",
  "gene": "UniProtKB:O95361"
}